{
  "gene_symbol": "SLC12A2",
  "term_label": "chloride transmembrane transport",
  "term_id": "GO:1902476",
  "gene": "UniProtKB:P55011",
  "gene_name": "Solute carrier family 12 member 2"
}